{
  "gene": "UniProtKB:Q2KHT4",
  "gene_symbol": "GSG1",
  "term_label": "Unknown molecular function",
  "term_id": "UNKNOWN:0001",
  "gene_name": "Germ cell-specific gene 1 protein"
}